general adaptation syndrome [GO:0051866] (biological process) Relationships: is a type of multicellular organismal response to stress [GO:0033555] Definition: General adaptation syndrome is the set of changes in various organ systems of the body, especially the pituitary-endocrine system, in response to a wide range of strong external stimuli, both physiological and psychological. It is described as having three stages: alarm reaction, where the body detects the external stimulus; adaptation, where the body engages defensive countermeasures against the stressor; and exhaustion, where the body begins to run out of defenses. References: PMID:14847556 Sources: Wikipedia:General_adaptation_syndrome Also known as: general adaptation syndrome, physiological process, general adaptation syndrome, physiological response, physiological process during general adaptation syndrome, physiological response during general adaptation syndrome